{
  "gene_name": "Myeloid leukemia factor 1",
  "term_id": "GO:0006355",
  "gene": "UniProtKB:P58340",
  "term_label": "regulation of DNA-templated transcription",
  "gene_symbol": "MLF1"
}